{
  "term_id": "GO:0032926",
  "term_label": "negative regulation of activin receptor signaling pathway",
  "gene": "UniProtKB:O95633",
  "gene_name": "Follistatin-related protein 3",
  "gene_symbol": "FSTL3"
}